{
  "gene": "UniProtKB:Q96A58",
  "gene_name": "Ras-related and estrogen-regulated growth inhibitor",
  "term_label": "GTPase activity",
  "gene_symbol": "RERG",
  "term_id": "GO:0003924"
}